{
  "term_label": "nucleus",
  "gene": "UniProtKB:Q9UJW3",
  "gene_symbol": "DNMT3L",
  "gene_name": "DNA (cytosine-5)-methyltransferase 3-like",
  "term_id": "GO:0005634"
}